{
  "gene_symbol": "BAIAP3",
  "term_label": "positive regulation of neurotransmitter secretion",
  "term_id": "GO:0001956",
  "gene": "UniProtKB:O94812",
  "gene_name": "BAI1-associated protein 3"
}